{
  "gene_name": "Matrix metalloproteinase-20",
  "term_label": "Unknown cellular component",
  "gene_symbol": "MMP20",
  "term_id": "UNKNOWN:0003",
  "gene": "UniProtKB:O60882"
}